metanephric mesenchymal cell migration [GO:0035789] (biological process) Definition: The orderly movement of undifferentiated metanephric mesenchymal cells (precursors to metanephric mesangial cells) from the mesenchyme into the cleft of the developing glomerulus, during development of the metanephros. Relationships: is a type of cell migration involved in metanephros development [GO:0035788] References: PMID:10734101, PMID:19019919 Sources: GOC:bf, GOC:mtg_kidney_jan10, GOC:yaf Regulation: regulated by GO:2000589; negatively regulated by negative regulation of metanephric mesenchymal cell migration [GO:2000590]; positively regulated by positive regulation of metanephric mesenchymal cell migration [GO:2000591] Also known as: metanephric mesenchyme chemotaxis